pancreas morphogenesis [GO:0061113] (biological process) Definition: Morphogenesis of the pancreas. Morphogenesis is the process in which anatomical structures are generated and organized. Sources: GOC:dph Relationships: is a type of GO:0009887; is part of pancreas development [GO:0031016]